{
  "term_id": "GO:0005634",
  "term_label": "nucleus",
  "gene_symbol": "ZNF324B",
  "gene_name": "Zinc finger protein 324B",
  "gene": "UniProtKB:Q6AW86"
}